Arp2/3 protein complex [GO:0005885] (cellular component) References: PMID:12479800 Sources: GOC:jl, GOC:vw Definition: A stable protein complex that contains two actin-related proteins, Arp2 and Arp3, and five novel proteins (ARPC1-5), and functions in the nucleation of branched actin filaments. Relationships: is a type of protein-containing complex [GO:0032991]; is part of actin cytoskeleton [GO:0015629]